{
  "term_id": "GO:0005634",
  "gene_symbol": "EEF1E1",
  "gene": "UniProtKB:O43324",
  "gene_name": "Eukaryotic translation elongation factor 1 epsilon-1",
  "term_label": "nucleus"
}